aggregation involved in sorocarp development [GO:0031152] (BP) Sources: GOC:mah, GOC:mtg_sensu, ISBN:0521583640 Relationships: is a type of cellular response to starvation [GO:0009267]; is a type of socially cooperative development [GO:0099120]; is part of sorocarp development [GO:0030587] Regulation: regulated by GO:0060176; positively regulated by GO:0110013; negatively regulated by GO:0110014 Definition: The process whose specific outcome is the progression of the aggregate over time, from its formation to the point when a slug is formed. Aggregate development begins in response to starvation and continues by the chemoattractant-mediated movement of cells toward each other. The aggregate is a multicellular structure that gives rise to the slug. Also known as: aggregate development involved in sorocarp development, aggregation during fruiting body development